{
  "term_id": "GO:0070552",
  "gene_symbol": "BRCC3",
  "term_label": "BRISC complex",
  "gene_name": "Lys-63-specific deubiquitinase BRCC36",
  "gene": "UniProtKB:P46736"
}